{
  "gene": "UniProtKB:Q86UX6",
  "term_id": "GO:0004674",
  "gene_name": "Serine_threonine-protein kinase 32C",
  "term_label": "protein serine/threonine kinase activity",
  "gene_symbol": "STK32C"
}